{
  "gene_symbol": "PSG6",
  "term_label": "Unknown molecular function",
  "term_id": "UNKNOWN:0001",
  "gene_name": "Pregnancy-specific beta-1-glycoprotein 6",
  "gene": "UniProtKB:Q00889"
}